{
  "gene": "UniProtKB:P27540",
  "gene_symbol": "ARNT",
  "gene_name": "Aryl hydrocarbon receptor nuclear translocator",
  "term_id": "GO:0000978",
  "term_label": "RNA polymerase II cis-regulatory region sequence-specific DNA binding"
}